{
  "term_id": "GO:0120193",
  "gene_symbol": "CLDN19",
  "term_label": "tight junction organization",
  "gene_name": "Claudin-19",
  "gene": "UniProtKB:Q8N6F1"
}